{
  "gene_name": "Cullin-7",
  "gene": "UniProtKB:Q14999",
  "term_id": "GO:0031467",
  "gene_symbol": "CUL7",
  "term_label": "Cul7-RING ubiquitin ligase complex"
}